positive regulation of Wnt signaling pathway [GO:0030177] (biological process) Relationships: is a type of positive regulation of signal transduction [GO:0009967]; is a type of regulation of Wnt signaling pathway [GO:0030111]; positively regulates GO:0016055 Sources: GOC:dph, GOC:go_curators, GOC:tb Subtypes: GO:0090263, positive regulation of non-canonical Wnt signaling pathway [GO:2000052] Also known as: positive regulation of Wnt receptor signaling pathway, positive regulation of Wnt receptor signalling pathway, positive regulation of Wnt-activated signaling pathway, positive regulation of frizzled signaling pathway, positive regulation of frizzled signalling pathway, up regulation of Wnt receptor signaling pathway, up regulation of frizzled signaling pathway, up-regulation of Wnt receptor signaling pathway, up-regulation of frizzled signaling pathway, upregulation of Wnt receptor signaling pathway, upregulation of frizzled signaling pathway, activation of Wnt receptor signaling pathway, activation of frizzled signaling pathway, stimulation of Wnt receptor signaling pathway, stimulation of frizzled signaling pathway Definition: Any process that activates or increases the frequency, rate or extent of Wnt signal transduction.